{
  "term_label": "Unknown molecular function",
  "gene_symbol": "ZNF41",
  "gene_name": "Zinc finger protein 41",
  "gene": "UniProtKB:P51814",
  "term_id": "UNKNOWN:0001"
}